{
  "gene": "UniProtKB:O60234",
  "gene_symbol": "GMFG",
  "term_label": "Arp2/3 complex binding",
  "term_id": "GO:0071933",
  "gene_name": "Glia maturation factor gamma"
}